paramyosin filament assembly or disassembly [GO:0061204] (biological process) Subtypes: striated muscle paramyosin thick filament assembly [GO:0061203] Relationships: is a type of actin cytoskeleton organization [GO:0030036] Sources: GOC:dph, GOC:kmv Definition: The formation or disassembly of a filament composed of paramyosin molecules.